{
  "gene": "UniProtKB:Q9UHF4",
  "gene_name": "Interleukin-20 receptor subunit alpha",
  "gene_symbol": "IL20RA",
  "term_label": "plasma membrane",
  "term_id": "GO:0005886"
}